aldehyde dehydrogenase [NAD(P)+] activity [GO:0004030] (molecular function) Definition: Catalysis of the reaction: an aldehyde + NAD(P)+ + H2O = an acid + NAD(P)H + H+. Sources: EC:1.2.1.5 Also known as: ALDH, aldehyde:NAD(P)+ oxidoreductase activity Relationships: is a type of oxidoreductase activity, acting on the aldehyde or oxo group of donors, NAD or NADP as acceptor [GO:0016620] Subtypes: GO:0004029, GO:0004043, aldehyde dehydrogenase (NADP+) activity [GO:0033721], butanal dehydrogenase [NAD(P)+] activity [GO:0047759], GO:0050269